{
  "term_label": "RNA polymerase II transcription regulatory region sequence-specific DNA binding",
  "gene_name": "Zinc finger protein 768",
  "term_id": "GO:0000977",
  "gene": "UniProtKB:Q9H5H4",
  "gene_symbol": "ZNF768"
}